{
  "gene": "UniProtKB:Q6PJE2",
  "gene_symbol": "POMZP3",
  "term_label": "Unknown cellular component",
  "term_id": "UNKNOWN:0003",
  "gene_name": "POM121 and ZP3 fusion protein"
}